{
  "term_label": "immune response-inhibiting cell surface receptor signaling pathway",
  "gene_name": "Killer cell immunoglobulin-like receptor 2DL5A",
  "gene": "UniProtKB:Q8N109",
  "gene_symbol": "KIR2DL5A",
  "term_id": "GO:0002767"
}